{
  "gene_name": "Homeobox protein aristaless-like 4",
  "term_label": "RNA polymerase II transcription regulatory region sequence-specific DNA binding",
  "term_id": "GO:0000977",
  "gene": "UniProtKB:Q9H161",
  "gene_symbol": "ALX4"
}